{
  "gene_symbol": "FAM201A",
  "term_label": "Unknown biological process",
  "gene": "UniProtKB:Q5SY85",
  "gene_name": "Protein FAM201A",
  "term_id": "UNKNOWN:0002"
}